{
  "gene": "UniProtKB:Q8NBZ7",
  "term_id": "GO:0005737",
  "gene_name": "UDP-glucuronic acid decarboxylase 1",
  "term_label": "cytoplasm",
  "gene_symbol": "UXS1"
}